{
  "gene_name": "Proteinase-activated receptor 1",
  "term_label": "thrombin-activated receptor activity",
  "gene": "UniProtKB:P25116",
  "term_id": "GO:0015057",
  "gene_symbol": "F2R"
}